{
  "gene_symbol": "HSP90AB3P",
  "term_id": "GO:0048471",
  "gene_name": "Putative heat shock protein HSP 90-beta-3",
  "gene": "UniProtKB:Q58FF7",
  "term_label": "perinuclear region of cytoplasm"
}